negative regulation of vascular associated smooth muscle cell dedifferentiation [GO:1905175] (biological process) Definition: Any process that stops, prevents or reduces the frequency, rate or extent of vascular smooth muscle cell dedifferentiation. References: PMID:19088079 Sources: GOC:BHF, GOC:BHF_miRNA, GOC:TermGenie, GOC:rph, GO_REF:0000058 Also known as: down regulation of vascular smooth muscle cell dedifferentiation, down-regulation of vascular smooth muscle cell dedifferentiation, downregulation of vascular smooth muscle cell dedifferentiation, negative regulation of vascular smooth muscle cell dedifferentiation, inhibition of vascular smooth muscle cell dedifferentiation Relationships: is a type of negative regulation of cellular process [GO:0048523]; is a type of negative regulation of developmental process [GO:0051093]; is a type of regulation of vascular associated smooth muscle cell dedifferentiation [GO:1905174]; negatively regulates vascular associated smooth muscle cell dedifferentiation [GO:1990936]